{
  "gene_name": "Heme transporter FLVCR2",
  "gene_symbol": "FLVCR2",
  "gene": "UniProtKB:Q9UPI3",
  "term_label": "heme binding",
  "term_id": "GO:0020037"
}